{
  "term_id": "GO:0010821",
  "term_label": "regulation of mitochondrion organization",
  "gene_name": "Presenilin-associated rhomboid-like protein, mitochondrial",
  "gene_symbol": "PARL",
  "gene": "UniProtKB:Q9H300"
}